anal fin morphogenesis [GO:0035144] (biological process) Definition: The process in which the anatomical structures of the anal fin are generated and organized. An anal fin is an unpaired medial fin on the ventral aspect near the caudal end of a fish, which provides lateral stability while swimming. Sources: GOC:dgh Relationships: is a type of medial fin morphogenesis [GO:0035141]; is part of GO:0033335 Subtypes: embryonic anal fin morphogenesis [GO:0035125], post-embryonic anal fin morphogenesis [GO:0035135]